{
  "gene_symbol": "ART1",
  "term_id": "UNKNOWN:0003",
  "term_label": "Unknown cellular component",
  "gene_name": "GPI-linked NAD(P)(+)--arginine ADP-ribosyltransferase 1",
  "gene": "UniProtKB:P52961"
}